{
  "term_id": "GO:0001817",
  "gene_symbol": "PLAGL1",
  "term_label": "regulation of cytokine production",
  "gene_name": "Zinc finger protein PLAGL1",
  "gene": "UniProtKB:Q9UM63"
}